{
  "term_label": "DNA-binding transcription factor activity, RNA polymerase II-specific",
  "term_id": "GO:0000981",
  "gene_symbol": "MKX",
  "gene": "UniProtKB:Q8IYA7",
  "gene_name": "Homeobox protein Mohawk"
}